{
  "gene": "UniProtKB:Q16820",
  "term_label": "extracellular space",
  "gene_symbol": "MEP1B",
  "gene_name": "Meprin A subunit beta",
  "term_id": "GO:0005615"
}